{
  "gene_name": "Olfactory receptor 5D16",
  "gene_symbol": "OR5D16",
  "term_label": "olfactory receptor activity",
  "term_id": "GO:0004984",
  "gene": "UniProtKB:Q8NGK9"
}